{
  "gene": "UniProtKB:Q86XT9",
  "gene_name": "Insulin-like growth factor-binding protein 3 receptor",
  "term_label": "Unknown molecular function",
  "gene_symbol": "TMEM219",
  "term_id": "UNKNOWN:0001"
}